Cvt vesicle assembly [GO:0071255] (BP) Definition: A vesicle organization process that takes place as part of the Cvt pathway, and results in the formation of a double membrane-bounded cytosolic structure that sequesters precursor aminopeptidase I (prAPI). Also known as: Cvt vesicle formation, cytoplasm to vacuole targeting vesicle assembly, cytoplasm-to-vacuole targetin vesicle assembly, Cvt vesicle biosynthesis References: PMID:10966461, PMID:11085977 Sources: GOC:rb Relationships: is a type of vesicle organization [GO:0016050]; is_a organelle assembly [GO:0070925]; BFO_0000050 GO:0032258